{
  "gene_symbol": "CACNG5",
  "gene": "UniProtKB:Q9UF02",
  "term_label": "voltage-gated calcium channel activity",
  "term_id": "GO:0005245",
  "gene_name": "Voltage-dependent calcium channel gamma-5 subunit"
}